positive regulation of ubiquitin-protein transferase activity [GO:0051443] (BP) Definition: Any process that activates, maintains or increases the rate of ubiquitin transferase activity. Also known as: positive regulation of ubiquitin transferase activity, up-regulation of ubiquitin transferase activity, upregulation of ubiquitin transferase activity, APC activation, APC activator, SCF complex activator, activation of ubiquitin transferase activity, anaphase promoting complex activator, anaphase-promoting complex activator, stimulation of ubiquitin transferase activity, ubiquitin transferase activator, up regulation of ubiquitin ligase activity Sources: GOC:ai, GOC:tb Subtypes: GO:1904668 Relationships: is a type of GO:0031398; is_a positive regulation of catalytic activity [GO:0043085]; is a type of regulation of ubiquitin-protein transferase activity [GO:0051438]; positively regulates GO:0004842